{
  "gene": "UniProtKB:Q9UMS6",
  "term_id": "GO:0005634",
  "gene_name": "Synaptopodin-2",
  "gene_symbol": "SYNPO2",
  "term_label": "nucleus"
}